2-C-methyl-D-erythritol 4-phosphate cytidylyltransferase activity [GO:0050518] (molecular function) Sources: EC:2.7.7.60, RHEA:13429 Also known as: 4-diphosphocytidyl-2C-methyl-D-erythritol synthase activity, CTP:2-C-methyl-D-erythritol 4-phosphate cytidylyltransferase activity, MEP cytidylyltransferase activity, 4-diphosphocytidyl-2-C-methyl-D-erythritol synthase activity, MCT activity Definition: Catalysis of the reaction: 2-C-methyl-D-erythritol 4-phosphate + CTP = 4-CDP-2-C-methyl-D-erythritol + diphosphate. Relationships: is_a cytidylyltransferase activity [GO:0070567]